L-ascorbate 6-phosphate lactonase activity [GO:0035460] (MF) References: PMID:18097099, PMID:20359483 Definition: Catalysis of the reaction: L-ascorbate 6-phosphate + H2O = 3-keto-L-gulonate 6-phosphate. Relationships: is a type of carboxylic ester hydrolase activity [GO:0052689]